male meiosis I [GO:0007141] (biological process) Sources: GOC:dph, GOC:mah Definition: A cell cycle process comprising the steps by which a cell progresses through male meiosis I, the first meiotic division in the male germline. Relationships: is a type of meiosis I [GO:0007127]; is a type of GO:0007140 Also known as: male meiosis I nuclear division